mitochondrial translational initiation [GO:0070124] (biological process) Sources: GOC:mah Regulation: regulated by regulation of mitochondrial translational initiation [GO:0070132]; negatively regulated by negative regulation of mitochondrial translational initiation [GO:0070133]; positively regulated by positive regulation of mitochondrial translational initiation [GO:0070134] Definition: The process preceding formation of the peptide bond between the first two amino acids of a protein in a mitochondrion. This includes the formation of a complex of the ribosome, mRNA, and an initiation complex that contains the first aminoacyl-tRNA. Also known as: mitochondrial translation initiation Relationships: is a type of translational initiation [GO:0006413]; BFO_0000050 GO:0032543; BFO_0000066 mitochondrion [GO:0005739]